response to acetaldehyde [GO:1905640] (BP) Relationships: is a type of response to oxygen-containing compound [GO:1901700] Definition: Any process that results in a change in state or activity of a cell or an organism (in terms of movement, secretion, enzyme production, gene expression, etc.) as a result of an acetaldehyde stimulus. References: PMID:27687866 Sources: GOC:TermGenie, GO_REF:0000071 Subtypes: GO:1905641